{
  "term_label": "protein localization to Golgi membrane",
  "gene_name": "Ras-related protein Rab-41",
  "gene": "UniProtKB:Q5JT25",
  "term_id": "GO:1903292",
  "gene_symbol": "RAB41"
}